{
  "gene": "UniProtKB:O94973",
  "term_id": "GO:0072583",
  "gene_name": "AP-2 complex subunit alpha-2",
  "gene_symbol": "AP2A2",
  "term_label": "clathrin-dependent endocytosis"
}